{
  "gene": "UniProtKB:Q8N695",
  "gene_symbol": "SLC5A8",
  "term_label": "Unknown cellular component",
  "term_id": "UNKNOWN:0003",
  "gene_name": "Sodium-coupled monocarboxylate transporter 1"
}